{
  "term_label": "Unknown cellular component",
  "gene_name": "E3 ubiquitin-protein ligase SH3RF3",
  "gene_symbol": "SH3RF3",
  "term_id": "UNKNOWN:0003",
  "gene": "UniProtKB:Q8TEJ3"
}